{
  "term_label": "plasma membrane",
  "term_id": "GO:0005886",
  "gene_symbol": "PXK",
  "gene_name": "PX domain-containing protein kinase-like protein",
  "gene": "UniProtKB:Q7Z7A4"
}